{
  "gene_symbol": "GATD1",
  "term_label": "cytoplasm",
  "term_id": "GO:0005737",
  "gene": "UniProtKB:Q8NB37",
  "gene_name": "Glutamine amidotransferase-like class 1 domain-containing protein 1"
}